negative regulation of interleukin-27 production [GO:0032711] (biological process) Definition: Any process that stops, prevents, or reduces the frequency, rate, or extent of interleukin-27 production. Sources: GOC:mah Also known as: down regulation of interleukin-27 production, down-regulation of interleukin-27 production, downregulation of interleukin-27 production, negative regulation of IL-27 production, inhibition of interleukin-27 production, negative regulation of interleukin-27 biosynthetic process Relationships: is a type of GO:0001818; is_a regulation of interleukin-27 production [GO:0032671]; negatively regulates interleukin-27 production [GO:0032631]